{
  "gene_symbol": "UPK3A",
  "gene_name": "Uroplakin-3a",
  "term_label": "plasma membrane",
  "term_id": "GO:0005886",
  "gene": "UniProtKB:O75631"
}